{
  "gene_name": "CCN family member 2",
  "term_label": "positive regulation of cell differentiation",
  "term_id": "GO:0045597",
  "gene_symbol": "CCN2",
  "gene": "UniProtKB:P29279"
}